{
  "term_label": "cyclin-dependent protein serine/threonine kinase activity",
  "gene_symbol": "CDK1",
  "gene_name": "Cyclin-dependent kinase 1",
  "gene": "UniProtKB:P06493",
  "term_id": "GO:0004693"
}